{
  "term_id": "GO:0043197",
  "gene_symbol": "APBA2",
  "term_label": "dendritic spine",
  "gene": "UniProtKB:Q99767",
  "gene_name": "Amyloid-beta A4 precursor protein-binding family A member 2"
}